{
  "term_id": "GO:0003725",
  "gene": "UniProtKB:Q9UL40",
  "gene_name": "Zinc finger protein 346",
  "gene_symbol": "ZNF346",
  "term_label": "double-stranded RNA binding"
}